acyl-glucuronidase activity [GO:0036237] (MF) References: PMID:22294686 Sources: GOC:BHF, GOC:vk Relationships: is_a glucuronidase activity [GO:0046574] Definition: Catalysis of the reaction: an acyl-glucuronoside + H2O = an alcohol + D-glucuronate. Also known as: acyl-glucuronide deglucuronidation activity